{
  "term_label": "endoplasmic reticulum membrane",
  "gene_symbol": "LMF1",
  "term_id": "GO:0005789",
  "gene": "UniProtKB:Q96S06",
  "gene_name": "Lipase maturation factor 1"
}